{
  "term_label": "nucleus",
  "gene_name": "Probable RNA-binding protein 46",
  "term_id": "GO:0005634",
  "gene_symbol": "RBM46",
  "gene": "UniProtKB:Q8TBY0"
}